{
  "term_label": "inflammatory response",
  "gene_name": "C-C motif chemokine 7",
  "term_id": "GO:0006954",
  "gene": "UniProtKB:P80098",
  "gene_symbol": "CCL7"
}